{
  "gene_symbol": "PIK3R6",
  "term_label": "G protein-coupled receptor signaling pathway",
  "gene_name": "Phosphoinositide 3-kinase regulatory subunit 6",
  "term_id": "GO:0007186",
  "gene": "UniProtKB:Q5UE93"
}